{
  "gene_symbol": "BCL2L1",
  "gene": "UniProtKB:Q07817",
  "term_label": "release of cytochrome c from mitochondria",
  "gene_name": "Bcl-2-like protein 1",
  "term_id": "GO:0001836"
}